regulation of skeletal muscle tissue development [GO:0048641] (biological process) Subtypes: regulation of branchiomeric skeletal muscle development [GO:0014711], GO:0014725, negative regulation of skeletal muscle tissue development [GO:0048642], positive regulation of skeletal muscle tissue development [GO:0048643] Definition: Any process that modulates the frequency, rate or extent of skeletal muscle tissue development. Relationships: is a type of regulation of striated muscle tissue development [GO:0016202]; RO_0002211 skeletal muscle tissue development [GO:0007519] Sources: GOC:go_curators